{
  "gene_symbol": "CLASRP",
  "term_id": "UNKNOWN:0003",
  "gene": "UniProtKB:Q8N2M8",
  "gene_name": "CLK4-associating serine_arginine rich protein",
  "term_label": "Unknown cellular component"
}